{
  "term_id": "UNKNOWN:0002",
  "term_label": "Unknown biological process",
  "gene_name": "Tetraspanin-3",
  "gene_symbol": "TSPAN3",
  "gene": "UniProtKB:O60637"
}